{
  "term_label": "axoneme",
  "gene_name": "Dynein axonemal heavy chain 11",
  "gene": "UniProtKB:Q96DT5",
  "term_id": "GO:0005930",
  "gene_symbol": "DNAH11"
}